{
  "gene_symbol": "KIAA0930",
  "gene_name": "Uncharacterized protein KIAA0930",
  "term_id": "UNKNOWN:0003",
  "term_label": "Unknown cellular component",
  "gene": "UniProtKB:Q6ICG6"
}